{
  "gene_symbol": "KLK5",
  "gene": "UniProtKB:Q9Y337",
  "term_label": "extracellular matrix disassembly",
  "term_id": "GO:0022617",
  "gene_name": "Kallikrein-5"
}